{
  "gene_name": "Syntaxin-16",
  "gene": "UniProtKB:O14662",
  "term_label": "SNAP receptor activity",
  "term_id": "GO:0005484",
  "gene_symbol": "STX16"
}